{
  "term_label": "Unknown biological process",
  "gene_symbol": "TMEM163",
  "gene": "UniProtKB:Q8TC26",
  "term_id": "UNKNOWN:0002",
  "gene_name": "Transmembrane protein 163"
}